{
  "gene_symbol": "MTHFD1",
  "gene_name": "C-1-tetrahydrofolate synthase, cytoplasmic",
  "term_id": "GO:0005829",
  "term_label": "cytosol",
  "gene": "UniProtKB:P11586"
}